positive regulation of exocytosis [GO:0045921] (biological process) Definition: Any process that activates or increases the frequency, rate or extent of exocytosis. Sources: GOC:go_curators Also known as: up regulation of exocytosis, up-regulation of exocytosis, upregulation of exocytosis, activation of exocytosis, stimulation of exocytosis Relationships: is a type of regulation of exocytosis [GO:0017157]; is a type of positive regulation of secretion by cell [GO:1903532]; positively regulates exocytosis [GO:0006887] Subtypes: positive regulation of regulated secretory pathway [GO:1903307], GO:1903435, positive regulation of exosomal secretion [GO:1903543]